{
  "term_id": "GO:0008312",
  "gene_name": "Signal recognition particle subunit SRP72",
  "term_label": "7S RNA binding",
  "gene_symbol": "SRP72",
  "gene": "UniProtKB:O76094"
}